{
  "term_label": "RNA polymerase II cis-regulatory region sequence-specific DNA binding",
  "gene_name": "Forkhead box protein S1",
  "gene": "UniProtKB:O43638",
  "term_id": "GO:0000978",
  "gene_symbol": "FOXS1"
}